{
  "gene_symbol": "SPOUT1",
  "term_label": "mitotic spindle",
  "gene": "UniProtKB:Q5T280",
  "gene_name": "Putative methyltransferase C9orf114",
  "term_id": "GO:0072686"
}